butyrate-acetoacetate CoA-transferase activity [GO:0047371] (molecular function) Also known as: butanoyl-CoA:acetoacetate CoA-transferase activity, butyryl coenzyme A-acetoacetate coenzyme A-transferase activity, butyryl-CoA-acetoacetate CoA-transferase activity Relationships: is a type of GO:0008410 Definition: Catalysis of the reaction: acetoacetate + butanoyl-CoA = acetoacetyl-CoA + butanoate. Sources: EC:2.8.3.9, RHEA:12961